positive regulation of cellular response to gamma radiation [GO:1905845] (biological process) Relationships: is a type of positive regulation of cellular process [GO:0048522]; is a type of regulation of cellular response to gamma radiation [GO:1905843]; is_a positive regulation of response to gamma radiation [GO:2001230]; positively regulates cellular response to gamma radiation [GO:0071480] References: PMID:23505386 Sources: GOC:TermGenie, GO_REF:0000058 Also known as: up regulation of cellular response to gamma radiation, up-regulation of cellular response to gamma radiation, upregulation of cellular response to gamma radiation, activation of cellular response to gamma radiation, activation of cellular response to gamma ray, activation of cellular response to gamma-ray photon, positive regulation of cellular response to gamma ray, positive regulation of cellular response to gamma-ray photon, up regulation of cellular response to gamma ray, up regulation of cellular response to gamma-ray photon, up-regulation of cellular response to gamma ray, up-regulation of cellular response to gamma-ray photon, upregulation of cellular response to gamma ray, upregulation of cellular response to gamma-ray photon Definition: Any process that activates or increases the frequency, rate or extent of cellular response to gamma radiation.